cation-transporting ATPase complex [GO:0090533] (cellular component) Subtypes: potassium:proton exchanging ATPase complex [GO:0005889], sodium:potassium-exchanging ATPase complex [GO:0005890], potassium ion-transporting ATPase complex [GO:0031004], proton-transporting V-type ATPase complex [GO:0033176], calcium ion-transporting ATPase complex [GO:0090534] Definition: Protein complex that carries out the reaction: ATP + H2O + cation(out) = ADP + phosphate + cation(in). Relationships: is a type of ATPase dependent transmembrane transport complex [GO:0098533] Sources: GOC:BHF